{
  "term_id": "GO:0045944",
  "gene": "UniProtKB:Q15365",
  "gene_name": "Poly(rC)-binding protein 1",
  "gene_symbol": "PCBP1",
  "term_label": "positive regulation of transcription by RNA polymerase II"
}